labyrinthine layer morphogenesis [GO:0060713] (biological process) Definition: The process in which the labyrinthine layer of the placenta is generated and organized. Sources: GOC:dph Relationships: is a type of embryonic morphogenesis [GO:0048598]; is part of embryonic placenta morphogenesis [GO:0060669]; is part of labyrinthine layer development [GO:0060711]